{
  "term_id": "GO:0006338",
  "gene_symbol": "PSIP1",
  "gene": "UniProtKB:O75475",
  "term_label": "chromatin remodeling",
  "gene_name": "PC4 and SFRS1-interacting protein"
}